{
  "gene": "UniProtKB:Q9UPQ0",
  "gene_symbol": "LIMCH1",
  "gene_name": "LIM and calponin homology domains-containing protein 1",
  "term_id": "GO:0032034",
  "term_label": "myosin II head/neck binding"
}